{
  "term_id": "GO:0005092",
  "gene_name": "G-protein-signaling modulator 2",
  "gene": "UniProtKB:P81274",
  "gene_symbol": "GPSM2",
  "term_label": "GDP-dissociation inhibitor activity"
}